negative regulation of mannotriose transport [GO:1900328] (biological process) Sources: GOC:TermGenie, GOC:mengo_curators Definition: Any process that stops, prevents or reduces the frequency, rate or extent of mannotriose transport. Relationships: is a type of GO:0051051; is_a regulation of mannotriose transport [GO:1900327]; negatively regulates GO:2001095 Also known as: down regulation of mannotriose transport, down-regulation of mannotriose transport, downregulation of mannotriose transport, inhibition of mannotriose transport